positive regulation of branching morphogenesis of a nerve [GO:1905492] (BP) References: PMID:16516839 Sources: GOC:TermGenie, GO_REF:0000058 Also known as: up regulation of branching morphogenesis of a nerve, up-regulation of branching morphogenesis of a nerve, upregulation of branching morphogenesis of a nerve, activation of branching morphogenesis of a nerve Relationships: is a type of positive regulation of developmental process [GO:0051094]; is a type of positive regulation of multicellular organismal process [GO:0051240]; is a type of regulation of branching morphogenesis of a nerve [GO:2000172]; positively regulates GO:0048755 Definition: Any process that activates or increases the frequency, rate or extent of branching morphogenesis of a nerve.